symbiont-mediated perturbation of host Rho small GTPase signal transduction [GO:0044083] (biological process) Definition: A process in which a symbiont alters a Rho protein family-mediated signal transduction pathway in its host organism. The host is defined as the larger of the organisms involved in a symbiotic interaction. Relationships: is a type of symbiont-mediated perturbation of host small GTPase-mediated signal transduction [GO:0044082] References: PMID:15694861, PMID:17689917, PMID:30201700 Also known as: modulation by symbiont of host Rho protein mediated signal transduction, modulation by symbiont of host Rho protein signal transduction, modulation by symbiont of host Rho protein-mediated signal transduction, modulation of host Rho protein signal transduction by symbiont, modulation of host Rho protein signaling by symbiont, modulation of host Rho protein signalling by symbiont, perturbation of host Rho protein signal transduction, regulation by symbiont of host Rho protein signal transduction, symbiont-mediated perturbation of host Rho protein signal transduction